{
  "gene": "UniProtKB:Q9NPE3",
  "gene_name": "H_ACA ribonucleoprotein complex subunit 3",
  "term_label": "snRNA pseudouridine synthesis",
  "term_id": "GO:0031120",
  "gene_symbol": "NOP10"
}